{
  "gene": "UniProtKB:Q96F07",
  "term_label": "synapse",
  "term_id": "GO:0045202",
  "gene_symbol": "CYFIP2",
  "gene_name": "Cytoplasmic FMR1-interacting protein 2"
}